{
  "gene_name": "Golgi-resident adenosine 3',5'-bisphosphate 3'-phosphatase",
  "gene_symbol": "BPNT2",
  "gene": "UniProtKB:Q9NX62",
  "term_id": "GO:0012505",
  "term_label": "endomembrane system"
}